symbiont-mediated perturbation of host cellular process [GO:0044068] (biological process) Definition: A process in which a symbiont alters or subverts a cellular biological process in its host organism. The host is defined as the larger of the organisms involved in a symbiotic interaction. Subtypes: symbiont-mediated transformation of host cell [GO:0019087], symbiont-mediated perturbation of host erythrocyte aggregation [GO:0020013], symbiont-mediated perturbation of host chromatin organization [GO:0039525], symbiont-mediated suppression of host peptidoglycan biosynthetic process [GO:0039635], symbiont-mediated suppression of host cell wall biogenesis [GO:0039636], symbiont-mediated perturbation of host cell cycle G0/G1 transition checkpoint [GO:0039646], symbiont-mediated perturbation of host ubiquitin-like protein modification [GO:0039648], symbiont-mediated perturbation of host gene expression [GO:0039656], symbiont-mediated perturbation of host natural killer cell mediated immune response [GO:0039671], symbiont-mediated perturbation of host cell cycle progression [GO:0044071], symbiont-mediated perturbation of host vacuole organization [GO:0044075], symbiont-mediated perturbation of host neurotransmitter secretion [GO:0044079], GO:0044542, symbiont-mediated perturbation of host synaptic transmission [GO:0044758], GO:0044865, symbiont-mediated induction of tumor or growth in host [GO:0051819], symbiont-mediated perturbation of host signal transduction pathway [GO:0052027], symbiont-mediated perturbation of host intracellular transport [GO:0052038], symbiont-mediated perturbation of host programmed cell death [GO:0052040], symbiont-mediated induction of syncytium formation [GO:0060141], symbiont-mediated perturbation of host autophagy [GO:0075071], symbiont-mediated suppression of host DNA replication [GO:0098673], symbiont-mediated disruption of host cell-cell adhesion [GO:0141023], symbiont-mediated suppression of host reactive oxygen species generation [GO:0141083], GO:0141145, symbiont-mediated suppression of host phagosome maturation [GO:0141158], symbiont-mediated perturbation of host cell motility [GO:1903653], symbiont-mediated perturbation of host vesicle-mediated transport [GO:1990215] Relationships: is a type of symbiont-mediated perturbation of host process [GO:0044003] Also known as: modulation by symbiont of host cellular process, modulation of host cellular process by symbiont, regulation by symbiont of host cellular process, regulation of host cellular process by symbiont Sources: MITRE:tk